{
  "gene_name": "Tubulin-specific chaperone A",
  "gene": "UniProtKB:O75347",
  "gene_symbol": "TBCA",
  "term_id": "GO:0006457",
  "term_label": "protein folding"
}